{
  "term_id": "GO:0001501",
  "term_label": "skeletal system development",
  "gene_name": "Collagen alpha-1(XVIII) chain",
  "gene_symbol": "COL18A1",
  "gene": "UniProtKB:P39060"
}